{
  "gene_symbol": "HUWE1",
  "gene": "UniProtKB:Q7Z6Z7",
  "term_id": "GO:0000139",
  "term_label": "Golgi membrane",
  "gene_name": "E3 ubiquitin-protein ligase HUWE1"
}